{
  "term_id": "GO:0003887",
  "gene": "UniProtKB:P06746",
  "term_label": "DNA-directed DNA polymerase activity",
  "gene_symbol": "POLB",
  "gene_name": "DNA polymerase beta"
}